{
  "gene_symbol": "AIP",
  "term_id": "UNKNOWN:0002",
  "term_label": "Unknown biological process",
  "gene": "UniProtKB:O00170",
  "gene_name": "AH receptor-interacting protein"
}